{
  "term_id": "GO:0006396",
  "gene": "UniProtKB:Q9GZR2",
  "gene_name": "RNA exonuclease 4",
  "term_label": "RNA processing",
  "gene_symbol": "REXO4"
}